activation of plasma proteins involved in acute inflammatory response [GO:0002541] (biological process) Regulation: positively regulated by Factor XII activation [GO:0002542] Definition: Any process activating plasma proteins by proteolysis as part of an acute inflammatory response. Relationships: is a type of GO:0016485; is part of acute inflammatory response [GO:0002526] Sources: GOC:jal, ISBN:0781735149